{
  "term_id": "UNKNOWN:0003",
  "gene_name": "Splicing factor 3B subunit 6",
  "term_label": "Unknown cellular component",
  "gene_symbol": "SF3B6",
  "gene": "UniProtKB:Q9Y3B4"
}